caudal fin development [GO:0033336] (biological process) Definition: The process whose specific outcome is the progression of the caudal fin over time, from its formation to the mature structure. Sources: GOC:dgh Relationships: is a type of medial fin development [GO:0033338]